{
  "gene_name": "Alpha-(1,3)-fucosyltransferase 11",
  "gene": "UniProtKB:Q495W5",
  "term_label": "Unknown biological process",
  "term_id": "UNKNOWN:0002",
  "gene_symbol": "FUT11"
}